CXCR chemokine receptor binding [GO:0045236] (molecular function) Also known as: alpha chemokine receptor binding, C-X-C chemokine receptor ligand, CXC chemokine receptor ligand, alpha chemokine receptor ligand References: PMID:11910892 Sources: GOC:ceb Relationships: is_a GO:0042379 Definition: Binding to a chemokine receptor in the CXCR family. Subtypes: interleukin-8 receptor binding [GO:0005153], CXCR4 chemokine receptor binding [GO:0031723], CXCR5 chemokine receptor binding [GO:0031724], CXCR6 chemokine receptor binding [GO:0031725], CXCR3 chemokine receptor binding [GO:0048248]